{
  "gene_symbol": "MCM9",
  "term_id": "GO:0017116",
  "term_label": "single-stranded DNA helicase activity",
  "gene": "UniProtKB:Q9NXL9",
  "gene_name": "DNA helicase MCM9"
}